otic vesicle morphogenesis [GO:0071600] (biological process) Regulation: regulated by regulation of otic vesicle morphogenesis [GO:1904118]; negatively regulated by negative regulation of otic vesicle morphogenesis [GO:1904119]; positively regulated by GO:1904120 Definition: The process in which the anatomical structures of the otic vesicle are generated and organized. The otic vesicle is a transient embryonic structure formed during development of the vertebrate inner ear. Sources: GOC:mah Relationships: is a type of inner ear morphogenesis [GO:0042472]; is a type of embryonic organ morphogenesis [GO:0048562]; is a type of epithelial tube morphogenesis [GO:0060562]; is part of otic vesicle development [GO:0071599]